juvenile hormone epoxide hydrolase activity [GO:0008096] (molecular function) Relationships: is a type of epoxide hydrolase activity [GO:0004301] Definition: Catalysis of the hydrolysis of the epoxide in a juvenile hormone to the corresponding diol. References: PMID:8396141 Sources: GOC:mah